positive regulation of CD8-positive, alpha-beta T cell activation [GO:2001187] (biological process) Relationships: is a type of GO:0046635; is a type of regulation of CD8-positive, alpha-beta T cell activation [GO:2001185]; positively regulates GO:0036037 Subtypes: positive regulation of CD8-positive, alpha-beta T cell differentiation [GO:0043378], positive regulation of CD8-positive, alpha-beta T cell proliferation [GO:2000566] Sources: GOC:obol Definition: Any process that activates or increases the frequency, rate or extent of CD8-positive, alpha-beta T cell activation.